extrinsic component of periplasmic side of plasma membrane [GO:0031236] (cellular component) Relationships: is a type of extrinsic component of external side of plasma membrane [GO:0031232]; is part of periplasmic side of plasma membrane [GO:0098567] Sources: GOC:dos, GOC:mah, GOC:mtg_sensu Also known as: extrinsic to external leaflet of plasma membrane, in periplasmic space, extrinsic to external side of plasma membrane, in periplasmic space Definition: The component of a plasma membrane consisting of gene products and protein complexes that are loosely bound to its periplasmic surface, but not integrated into the hydrophobic region.